{
  "term_id": "GO:0006297",
  "term_label": "nucleotide-excision repair, DNA gap filling",
  "gene": "UniProtKB:Q07864",
  "gene_symbol": "POLE",
  "gene_name": "DNA polymerase epsilon catalytic subunit A"
}